{
  "term_label": "protein serine/threonine kinase activity",
  "gene_name": "Serine_threonine-protein kinase pim-1",
  "gene_symbol": "PIM1",
  "term_id": "GO:0004674",
  "gene": "UniProtKB:P11309"
}